{
  "gene_name": "Host cell factor 2",
  "gene": "UniProtKB:Q9Y5Z7",
  "term_label": "histone methyltransferase complex",
  "term_id": "GO:0035097",
  "gene_symbol": "HCFC2"
}